sperm individualization [GO:0007291] (biological process) Definition: The resolution of the male germline syncytium or cyst into individual gametes by packaging each spermatid into its own plasma membrane. References: PMID:9550716 Sources: GOC:bf Relationships: is a type of developmental process involved in reproduction [GO:0003006]; is a type of cellularization [GO:0007349]; is part of GO:0007286